hexuronate transmembrane transporter activity [GO:0015134] (molecular function) Sources: GOC:ai, GOC:mtg_transport, ISBN:0198506732, ISBN:0815340729 Relationships: is a type of GO:0015133; is part of GO:0015736; is part of hexuronide transmembrane transport [GO:0015778] Also known as: hexuronide transmembrane transporter activity Definition: Enables the transfer of hexuronates from one side of a membrane to the other. A hexuronate is any monocarboxylic acid derived from a hexose by oxidation of C-6.